{
  "term_label": "nucleus",
  "gene": "UniProtKB:O95475",
  "term_id": "GO:0005634",
  "gene_name": "Homeobox protein SIX6",
  "gene_symbol": "SIX6"
}